{
  "gene": "UniProtKB:Q6ZXV5",
  "gene_name": "Protein O-mannosyl-transferase TMTC3",
  "gene_symbol": "TMTC3",
  "term_id": "GO:0005783",
  "term_label": "endoplasmic reticulum"
}